{
  "gene_symbol": "TOX",
  "gene_name": "Thymocyte selection-associated high mobility group box protein TOX",
  "term_id": "GO:0005634",
  "gene": "UniProtKB:O94900",
  "term_label": "nucleus"
}